regulation of pseurotin A biosynthetic process [GO:1900849] (BP) Definition: Any process that modulates the frequency, rate or extent of pseurotin A biosynthetic process. Sources: GOC:TermGenie, GOC:di Also known as: regulation of pseurotin A anabolism, regulation of pseurotin A biosynthesis, regulation of pseurotin A formation, regulation of pseurotin A synthesis, regulation of Pseurotin anabolism, regulation of Pseurotin biosynthesis, regulation of Pseurotin biosynthetic process, regulation of Pseurotin formation, regulation of Pseurotin synthesis Relationships: is a type of regulation of biosynthetic process [GO:0009889]; is_a regulation of amide metabolic process [GO:0034248]; is a type of regulation of small molecule metabolic process [GO:0062012]; regulates pseurotin A biosynthetic process [GO:1900790] Subtypes: negative regulation of pseurotin A biosynthetic process [GO:1900850], positive regulation of pseurotin A biosynthetic process [GO:1900851]